{
  "gene_name": "Synaptosomal-associated protein 25",
  "gene": "UniProtKB:P60880",
  "term_id": "GO:0005484",
  "gene_symbol": "SNAP25",
  "term_label": "SNAP receptor activity"
}